oxidative photosynthetic carbon pathway [GO:0009854] (biological process) Sources: ISBN:0943088399 Relationships: is a type of GO:0043094; BFO_0000050 photorespiration [GO:0009853] Definition: The reactions of the C2 pathway bring about the metabolic conversion of two molecules of 2-phosphoglycolate to one molecule of 3-phosphoglycerate, which can be used by the C3 cycle, and one molecule of carbon dioxide (CO2).